{
  "gene": "UniProtKB:Q8IZM9",
  "gene_name": "Probable sodium-coupled neutral amino acid transporter 6",
  "gene_symbol": "SLC38A6",
  "term_id": "GO:0003333",
  "term_label": "amino acid transmembrane transport"
}